trans-synaptic signaling by lipid, modulating synaptic transmission [GO:0099552] (biological process) Definition: Cell-cell signaling between presynapse and postsynapse, via the release and reception of lipid molecules, that modulates the synaptic transmission properties of the synapse. References: PMID:21531987 Sources: GOC:dos Note: Note that this term was created for the SynGO project, and will be obsoleted when the SynGO annotations are made in Noctua. Relationships: is a type of trans-synaptic signaling by lipid [GO:0099541]; is a type of trans-synaptic signaling, modulating synaptic transmission [GO:0099550] Subtypes: trans-synaptic signaling by endocannabinoid, modulating synaptic transmission [GO:0099553]